{
  "gene_name": "Keratin-associated protein 13-1",
  "term_label": "Unknown molecular function",
  "gene_symbol": "KRTAP13-1",
  "gene": "UniProtKB:Q8IUC0",
  "term_id": "UNKNOWN:0001"
}